positive regulation of immature T cell proliferation [GO:0033091] (biological process) Relationships: is a type of regulation of immature T cell proliferation [GO:0033083]; is a type of GO:0042102; positively regulates immature T cell proliferation [GO:0033079] Definition: Any process that activates or increases the frequency, rate or extent of immature T cell proliferation. Sources: GOC:add, GOC:mah Subtypes: positive regulation of immature T cell proliferation in thymus [GO:0033092]